{
  "term_label": "cholesterol biosynthetic process",
  "term_id": "GO:0006695",
  "gene": "UniProtKB:O15503",
  "gene_name": "Insulin-induced gene 1 protein",
  "gene_symbol": "INSIG1"
}